{
  "term_label": "extracellular matrix organization",
  "gene_name": "Stromelysin-3",
  "gene_symbol": "MMP11",
  "term_id": "GO:0030198",
  "gene": "UniProtKB:P24347"
}